high-affinity iron exporter complex [GO:0061841] (cellular component) References: PMID:10608875, PMID:9413439 Sources: GOC:bhm Definition: A protein complex which transports ferrous iron (Fe(III) or Fe3+) ions from the vacuole, the main storage component of intracellular free iron, into the cytoplasm in a low iron environment. Relationships: is a type of transmembrane transporter complex [GO:1902495]; is a type of ferroxidase complex [GO:1905862]; is part of vacuolar membrane [GO:0005774] Note: An example of this is FET5 in Saccharomyces cerevisiae (P43561) in PMID:9413439. Also known as: high affinity iron exporter complex, FET5-FTH1 high affinity iron exporter complex, FET5-FTH1 high-affinity iron exporter complex